H3-H4 histone complex chaperone activity [GO:0000510] (molecular function) Note: Mammalian cells have seven known sequence variants of histone H3. These are denoted as Histone H3.1, Histone H3.2, Histone H3.3, Histone H3.4 (H3T), Histone H3.5, Histone H3.X and Histone H3.Y (https://en.wikipedia.org/wiki/Histone_H3). Relationships: is a type of histone chaperone activity [GO:0140713] References: PMID:28053344 Definition: A histone chaperone that carries a H3-H4 histone complex. Also known as: H3-H4 histone carrier activity, H3.1-H4 histone complex chaperone activity, H3.2-H4 histone complex chaperone activity, H3.3-H4 histone complex chaperone activity Subtypes: GO:0140665